{
  "gene_name": "Plasminogen",
  "gene_symbol": "PLG",
  "term_label": "fibrinolysis",
  "gene": "UniProtKB:P00747",
  "term_id": "GO:0042730"
}